{
  "gene": "UniProtKB:Q6KF10",
  "term_label": "metanephros development",
  "gene_symbol": "GDF6",
  "gene_name": "Growth_differentiation factor 6",
  "term_id": "GO:0001656"
}